{
  "gene": "UniProtKB:C9JJH3",
  "term_id": "GO:0005634",
  "gene_symbol": "USP17L10",
  "term_label": "nucleus",
  "gene_name": "Ubiquitin carboxyl-terminal hydrolase 17-like protein 10"
}